hexokinase-dependent signaling [GO:0009747] (biological process) Definition: The series of molecular signals mediated by hexose and dependent on the detection of hexokinase. Relationships: is a type of hexose mediated signaling [GO:0009757] Also known as: hexokinase-dependent signalling Sources: GOC:mah, GOC:sm